neurotransmitter receptor cycle [GO:0099627] (biological process) Definition: The process during which neurotransmitter receptors, anchored in some region of the synaptic membrane, are recycled via the endosome. This cycle includes release from anchoring, diffusion in the synaptic membrane to an endocytic region, endocytosis, transport to the endosome, recycling in the endosome, transport back the synaptic membrane and subsequent anchoring (trapping). Subtypes: postsynaptic neurotransmitter receptor cycle [GO:0099630] Relationships: is a type of neurotransmitter receptor transport [GO:0099637] Sources: GOC:dos